arginine catabolic process to spermine [GO:0019548] (biological process) Relationships: is a type of GO:0006525; is a type of spermine metabolic process [GO:0008215]; is a type of alpha-amino acid catabolic process [GO:1901606] Definition: The chemical reactions and pathways resulting in the breakdown of arginine into other compounds, including spermine. Also known as: arginine breakdown to spermine, arginine degradation to spermine Sources: GOC:go_curators